synchronous neurotransmitter secretion [GO:0071911] (biological process) References: PMID:19477156, PMID:20643933 Sources: GOC:dsf Relationships: is a type of neurotransmitter secretion [GO:0007269] Definition: Release of neurotransmitter at the synapse that lasts for just a few milliseconds after action potential invasion.